{
  "term_id": "GO:0005886",
  "gene_symbol": "P2RY6",
  "gene": "UniProtKB:Q15077",
  "gene_name": "P2Y purinoceptor 6",
  "term_label": "plasma membrane"
}